{
  "gene_name": "FHF complex subunit HOOK-interacting protein 1B",
  "term_label": "Unknown molecular function",
  "term_id": "UNKNOWN:0001",
  "gene_symbol": "FHIP1B",
  "gene": "UniProtKB:Q8N612"
}